positive regulation of cardioblast proliferation [GO:1905062] (biological process) References: PMID:24236097 Sources: GOC:BHF, GOC:BHF_miRNA, GOC:TermGenie, GOC:bc, GO_REF:0000058 Definition: Any process that activates or increases the frequency, rate or extent of cardioblast proliferation. Relationships: is a type of regulation of cardioblast proliferation [GO:0003264]; is a type of positive regulation of cell proliferation involved in heart morphogenesis [GO:2000138]; positively regulates cardioblast proliferation [GO:0003263] Also known as: up regulation of cardioblast proliferation, up-regulation of cardioblast proliferation, upregulation of cardioblast proliferation, activation of cardioblast proliferation